nitrite reductase (NADPH) activity [GO:0106314] (molecular function) Definition: Catalysis of the reaction: ammonium hydroxide + 3 NADP+ + H2O = nitrite + 3 NADPH + 3 H+. Relationships: is a type of nitrite reductase [NAD(P)H] activity [GO:0008942] Sources: RHEA:24632